TBK1-IKKE-DDX3 complex [GO:0039658] (cellular component) References: PMID:18636090 Sources: VZ:719 Relationships: is a type of protein-containing complex [GO:0032991] Definition: A protein complex containing TBK1 (TANK-binding kinase 1), IKBKE (I-Kappa-B kinase epsilon/IKKE/IKK-epsilon) and the DEAD box family RNA helicase DDX3. Also known as: TBK1-IKBKE-DDX3 complex